{
  "term_label": "cytoplasm",
  "gene": "UniProtKB:A1L3X4",
  "gene_symbol": "MT1DP",
  "gene_name": "Putative metallothionein MT1DP",
  "term_id": "GO:0005737"
}